{
  "gene_name": "Keratin-associated protein 10-2",
  "gene": "UniProtKB:P60368",
  "term_id": "UNKNOWN:0002",
  "gene_symbol": "KRTAP10-2",
  "term_label": "Unknown biological process"
}